macrophage apoptotic process [GO:0071888] (BP) Also known as: macrophage apoptosis, AICD, activation-induced cell death Definition: Any apoptotic process in a macrophage, a mononuclear phagocyte present in a variety of tissues. Sources: CL:0000235, GOC:BHF, GOC:mah, GOC:mtg_apoptosis Note: Note that a lymphocyte is a cell of the B cell, T cell, or natural killer cell lineage (CL:0000542). Relationships: is a type of inflammatory cell apoptotic process [GO:0006925]; is a type of myeloid cell apoptotic process [GO:0033028]; is a type of GO:0071887 Regulation: regulated by regulation of macrophage apoptotic process [GO:2000109]; negatively regulated by negative regulation of macrophage apoptotic process [GO:2000110]; positively regulated by positive regulation of macrophage apoptotic process [GO:2000111]